Hedgehog signaling complex [GO:0035301] (cellular component) Definition: A multiprotein complex that binds microtubules in a Hedgehog-dependent manner, and is required for signal transduction by members of the Hedgehog family of proteins. The core components of the complex are the serine/threonine protein kinase Fused, the kinesin motor protein Costal2 (Cos2), and a zinc finger transcription factor (Gli family members in humans, and Cubitus interruptus (Ci) in Drosophila). References: PMID:10825151, PMID:15057936 Relationships: is a type of intracellular protein-containing complex [GO:0140535] Also known as: HSC, Hedgehog signalling complex